{
  "gene_name": "Phosphatidylcholine:ceramide cholinephosphotransferase 1",
  "gene": "UniProtKB:Q86VZ5",
  "gene_symbol": "SGMS1",
  "term_id": "GO:0005789",
  "term_label": "endoplasmic reticulum membrane"
}